{
  "gene_name": "Probable G-protein coupled receptor 33",
  "gene_symbol": "GPR33",
  "term_id": "GO:0007204",
  "term_label": "positive regulation of cytosolic calcium ion concentration",
  "gene": "UniProtKB:Q49SQ1"
}